{
  "term_label": "basolateral plasma membrane",
  "gene": "UniProtKB:Q96Q91",
  "gene_name": "Anion exchange protein 4",
  "gene_symbol": "SLC4A9",
  "term_id": "GO:0016323"
}